{
  "term_label": "oxidoreductase activity",
  "gene_name": "Lanosterol 14-alpha demethylase",
  "gene": "UniProtKB:Q16850",
  "gene_symbol": "CYP51A1",
  "term_id": "GO:0016491"
}